{
  "gene_symbol": "OR56B1",
  "gene": "UniProtKB:Q8NGI3",
  "term_id": "GO:0004984",
  "term_label": "olfactory receptor activity",
  "gene_name": "Olfactory receptor 56B1"
}